positive regulation of calcineurin-NFAT signaling cascade [GO:0070886] (biological process) Sources: GOC:mah Relationships: is a type of GO:0070884; is a type of positive regulation of calcineurin-mediated signaling [GO:0106058]; positively regulates GO:0033173 Definition: Any process that activates or increases the frequency, rate or extent of signaling via the calcineurin-NFAT signaling cascade. Also known as: positive regulation of calcineurin-NFAT signalling cascade, up regulation of calcineurin-NFAT signaling cascade, up-regulation of calcineurin-NFAT signaling cascade, upregulation of calcineurin-NFAT signaling cascade, activation of calcineurin-NFAT signaling cascade, positive regulation of NFAT protein import into nucleus, stimulation of calcineurin-NFAT signaling cascade, positive regulation of calcineurin-NFAT signaling pathway